{
  "gene": "UniProtKB:Q13698",
  "term_label": "voltage-gated calcium channel complex",
  "gene_symbol": "CACNA1S",
  "term_id": "GO:0005891",
  "gene_name": "Voltage-dependent L-type calcium channel subunit alpha-1S"
}